{
  "term_label": "angiogenesis",
  "gene": "UniProtKB:Q4VCS5",
  "gene_name": "Angiomotin",
  "term_id": "GO:0001525",
  "gene_symbol": "AMOT"
}